{
  "term_id": "GO:0030881",
  "gene_name": "HLA class I histocompatibility antigen, alpha chain F",
  "gene": "UniProtKB:P30511",
  "gene_symbol": "HLA-F",
  "term_label": "beta-2-microglobulin binding"
}